{
  "term_label": "DNA-binding transcription activator activity, RNA polymerase II-specific",
  "gene_symbol": "SOX21",
  "gene_name": "Transcription factor SOX-21",
  "gene": "UniProtKB:Q9Y651",
  "term_id": "GO:0001228"
}